{
  "gene_name": "Clusterin-like protein 1",
  "term_id": "GO:0005634",
  "gene": "UniProtKB:Q15846",
  "term_label": "nucleus",
  "gene_symbol": "CLUL1"
}